{
  "gene_name": "Centrosomal protein of 162 kDa",
  "gene_symbol": "CEP162",
  "term_label": "axonemal microtubule",
  "gene": "UniProtKB:Q5TB80",
  "term_id": "GO:0005879"
}